{
  "term_label": "Unknown biological process",
  "gene_symbol": "SPAG1",
  "term_id": "UNKNOWN:0002",
  "gene": "UniProtKB:Q07617",
  "gene_name": "Sperm-associated antigen 1"
}